RNA polymerase III transcription regulatory region sequence-specific DNA binding [GO:0001016] (MF) Subtypes: RNA polymerase III cis-regulatory region sequence-specific DNA binding [GO:0000992] Definition: Binding to a DNA region that controls the transcription of a gene by RNA polymerase III. Binding may occur as a sequence specific interaction or as an interaction observed only once a factor has been recruited to the DNA by other factors. Relationships: is a type of GO:0000976 References: PMID:12381659 Sources: GOC:txnOH, GOC:vw Also known as: RNA polymerase III regulatory region DNA binding